neuron projection guidance [GO:0097485] (biological process) Relationships: is a type of neuron projection development [GO:0031175]; is part of neuron projection morphogenesis [GO:0048812] References: PMID:22790009 Sources: GOC:BHF, GOC:rl Subtypes: axon guidance [GO:0007411], GO:0070983, GO:0097491 Also known as: neuron process guidance, neuron protrusion guidance, neuronal cell projection guidance, neurite guidance Definition: The process in which the migration of a neuron projection is directed to a specific target site in response to a combination of attractive and repulsive cues.